{
  "gene": "UniProtKB:Q9GZP7",
  "gene_name": "Vomeronasal type-1 receptor 1",
  "gene_symbol": "VN1R1",
  "term_label": "Unknown biological process",
  "term_id": "UNKNOWN:0002"
}